chromosomal DNA methylation maintenance following DNA replication [GO:0141119] (biological process) Definition: The process that maintains methylated cytosine in newly synthesized DNA following DNA replication. After the establishment of novel DNA methylation marks, the newly created patterns must be faithfully transmitted by maintenance DNA methyltransferases during cell division. References: PMID:11005794, PMID:20142834, PMID:26077819, PMID:34968368 Relationships: is_a GO:0006325 Note: CG methylation is maintained by two evolutionarily conserved core partners: (1) a maintenance DNA methyltransferase called DNMT1 in mammals and MET1 (DNA METHYLTRANSFERASE 1) in plants and (2) a cofactor named UHRF1 in mammals and VIM (VARIANT IN METHYLATION) in plants. In mammals, the maintenance of non-CG methylation typically involves DNMT3 enzymes. In plants, non-CG methylation is further divided in two classes of sequence, CHG and CHH, and requires distinct enzymatic machineries. Also known as: DNA methylation, DNA methylation maintenance, DNA methylation maintenance following DNA replication, DNA methylation maintenance following cell division, genome methylation maintenance following DNA replication